{
  "gene_symbol": "BAK1",
  "term_id": "GO:0043065",
  "gene": "UniProtKB:Q16611",
  "term_label": "positive regulation of apoptotic process",
  "gene_name": "Bcl-2 homologous antagonist_killer"
}